{
  "gene_name": "Glycophorin-E",
  "gene_symbol": "GYPE",
  "gene": "UniProtKB:P15421",
  "term_id": "GO:0005886",
  "term_label": "plasma membrane"
}